{
  "gene_name": "Lysine-specific demethylase 3B",
  "term_label": "transcription coregulator activity",
  "term_id": "GO:0003712",
  "gene_symbol": "KDM3B",
  "gene": "UniProtKB:Q7LBC6"
}